{
  "gene": "UniProtKB:Q8NGF4",
  "term_label": "sensory perception of smell",
  "term_id": "GO:0007608",
  "gene_symbol": "OR5AP2",
  "gene_name": "Olfactory receptor 5AP2"
}